{
  "gene_symbol": "IGFBP2",
  "term_id": "GO:0005615",
  "gene_name": "Insulin-like growth factor-binding protein 2",
  "term_label": "extracellular space",
  "gene": "UniProtKB:P18065"
}